{
  "term_id": "GO:1990414",
  "gene": "UniProtKB:O60216",
  "term_label": "replication-born double-strand break repair via sister chromatid exchange",
  "gene_symbol": "RAD21",
  "gene_name": "Double-strand-break repair protein rad21 homolog"
}